{
  "term_label": "Unknown molecular function",
  "term_id": "UNKNOWN:0001",
  "gene": "UniProtKB:Q75NE6",
  "gene_name": "Putative microRNA 17 host gene protein",
  "gene_symbol": "MIR17HG"
}